glutamate racemase activity [GO:0008881] (molecular function) Relationships: is a type of amino-acid racemase activity [GO:0047661] Sources: EC:5.1.1.3, RHEA:12813 Definition: Catalysis of the reaction: L-glutamate = D-glutamate.